radial spoke base [GO:0120339] (cellular component) Definition: The short portion of the radial spoke that is directly anchored to the A microtubule of an axonemal microtubule doublet. References: PMID:22754630, PMID:25694453 Sources: GOC:krc Relationships: is a type of GO:0032991; is part of GO:0001534 Subtypes: radial spoke base 1 [GO:0120340], GO:0120341, GO:0120342